{
  "gene_symbol": "MKKS",
  "term_label": "nucleus",
  "gene_name": "Molecular chaperone MKKS",
  "gene": "UniProtKB:Q9NPJ1",
  "term_id": "GO:0005634"
}